baicalin beta-D-glucuronidase activity [GO:0052748] (molecular function) Definition: Catalysis of the reaction: baicalin + H2O = baicalein + D-glucuronate. Sources: GOC:mengo_curators, RHEA:28130 Also known as: baicalinase activity, 5,6,7-trihydroxyflavone-7-O-beta-D-glucupyranosiduronate glucuronosylhydrolase activity Relationships: is a type of GO:0046574